{
  "term_label": "phosphatidylinositol-4,5-bisphosphate 5-phosphatase activity",
  "gene_symbol": "SYNJ2",
  "gene": "UniProtKB:O15056",
  "term_id": "GO:0004439",
  "gene_name": "Synaptojanin-2"
}